anther septum development [GO:0080128] (biological process) Sources: GOC:dhl, PO:0005010 Relationships: is a type of developmental process involved in reproduction [GO:0003006]; is a type of plant septum development [GO:1905328]; is part of anther development [GO:0048653] Definition: The process whose specific outcome is the progression of the anther septum over time, from its formation to the mature structure. The anther septum is a thin partition or stretch of cells that are present in the anther dehiscence zone.